{
  "term_label": "glutamate-cysteine ligase regulator activity",
  "gene_symbol": "GCLM",
  "term_id": "GO:1990609",
  "gene_name": "Glutamate--cysteine ligase regulatory subunit",
  "gene": "UniProtKB:P48507"
}